{
  "term_id": "GO:0000981",
  "gene_name": "Transcriptional repressor scratch 2",
  "gene": "UniProtKB:Q9NQ03",
  "term_label": "DNA-binding transcription factor activity, RNA polymerase II-specific",
  "gene_symbol": "SCRT2"
}